{
  "term_label": "endoplasmic reticulum to Golgi vesicle-mediated transport",
  "term_id": "GO:0006888",
  "gene_symbol": "STEEP1",
  "gene_name": "STING ER exit protein",
  "gene": "UniProtKB:Q9H5V9"
}